{
  "term_label": "cell surface receptor signaling pathway",
  "gene_name": "T-cell surface glycoprotein CD3 epsilon chain",
  "term_id": "GO:0007166",
  "gene_symbol": "CD3E",
  "gene": "UniProtKB:P07766"
}